{
  "gene_symbol": "GOLGA8R",
  "term_label": "Unknown molecular function",
  "gene_name": "Golgin subfamily A member 8R",
  "term_id": "UNKNOWN:0001",
  "gene": "UniProtKB:I6L899"
}